{
  "gene_symbol": "ATP1A1-AS1",
  "gene_name": "Putative uncharacterized protein ATP1A1-AS1",
  "gene": "UniProtKB:Q5TC04",
  "term_label": "Unknown cellular component",
  "term_id": "UNKNOWN:0003"
}